{
  "gene": "UniProtKB:Q96K31",
  "term_id": "UNKNOWN:0002",
  "gene_name": "Uncharacterized protein C8orf76",
  "term_label": "Unknown biological process",
  "gene_symbol": "C8orf76"
}